{
  "gene_symbol": "BSPH1",
  "term_label": "heparin binding",
  "gene": "UniProtKB:Q075Z2",
  "gene_name": "Binder of sperm protein homolog 1",
  "term_id": "GO:0008201"
}